oxidized purine DNA binding [GO:0032357] (molecular function) Sources: GOC:vk Subtypes: 8-hydroxy-2'-deoxyguanosine DNA binding [GO:1905773] Definition: Binding to a DNA region containing an oxidized purine residue. Also known as: oxidised purine DNA binding, oxidized purine base DNA binding, oxidized purine nucleobase DNA binding Relationships: is a type of GO:0032356